{
  "term_label": "protein autoubiquitination",
  "gene": "UniProtKB:Q7Z6J8",
  "term_id": "GO:0051865",
  "gene_name": "E3 ubiquitin-protein ligase E3D",
  "gene_symbol": "UBE3D"
}